{
  "gene": "UniProtKB:Q8NGA4",
  "gene_name": "Putative G-protein coupled receptor GPR32P1",
  "term_id": "GO:0006954",
  "term_label": "inflammatory response",
  "gene_symbol": "GPR32P1"
}